4-hydroxyacetophenone monooxygenase activity [GO:0033767] (molecular function) Definition: Catalysis of the reaction: 4'-hydroxyacetophenone + H+ + NADPH + O2 = 4-hydroxyphenyl acetate + H2O + NADP+. Relationships: is a type of oxidoreductase activity, acting on paired donors, with incorporation or reduction of molecular oxygen, NAD(P)H as one donor, and incorporation of one atom of oxygen [GO:0016709] Sources: EC:1.14.13.84, RHEA:22916 Also known as: (4-hydroxyphenyl)ethan-1-one,NADPH:oxygen oxidoreductase (ester-forming) activity, HAPMO